4-hydroxybenzoyl-CoA thioesterase activity [GO:0018739] (molecular function) Also known as: 4-hydroxybenzoyl-CoA thiolesterase activity, 4-hydroxybenzoyl-CoA hydrolase activity Sources: EC:3.1.2.23, RHEA:11948 Definition: Catalysis of the reaction: 4-hydroxybenzoyl-CoA + H2O = 4-hydroxybenzoate + CoA + H+. Relationships: is a type of acyl-CoA hydrolase activity [GO:0016289]